{
  "gene_symbol": "SMAP2",
  "gene_name": "Stromal membrane-associated protein 2",
  "term_label": "cytoplasm",
  "gene": "UniProtKB:Q8WU79",
  "term_id": "GO:0005737"
}